{
  "gene": "UniProtKB:Q58WW2",
  "term_label": "positive regulation of transcription by RNA polymerase II",
  "gene_symbol": "DCAF6",
  "term_id": "GO:0045944",
  "gene_name": "DDB1- and CUL4-associated factor 6"
}